proteinogenic amino acid metabolic process [GO:0170039] (biological process) Relationships: is a type of GO:0006520; is a type of carboxylic acid metabolic process [GO:0019752] Sources: GOC:ew Subtypes: glycine metabolic process [GO:0006544], L-histidine metabolic process [GO:0006547], L-leucine metabolic process [GO:0006551], GO:0006558, L-serine metabolic process [GO:0006563], L-tryptophan metabolic process [GO:0006568], tyrosine metabolic process [GO:0006570], glutamine family amino acid metabolic process [GO:0009064], 'de novo' NAD+ biosynthetic process from L-aspartate [GO:0034628], GO:0042851, L-cysteine metabolic process [GO:0046439], L-asparagine metabolic process [GO:0070982], proteinogenic amino acid biosynthetic process [GO:0170038], proteinogenic amino acid catabolic process [GO:0170040] Definition: The chemical reactions and pathways involving any amino acid that is incorporated into protein naturally by ribosomal translation of mRNA, and that has a specific codon for translation from mRNA to protein. Also known as: proteinogenic amino acid metabolism